{
  "gene_symbol": "IFNA1",
  "gene": "UniProtKB:P01562",
  "term_label": "type I interferon-mediated signaling pathway",
  "term_id": "GO:0060337",
  "gene_name": "Interferon alpha-1_13"
}